{
  "term_label": "immune response",
  "term_id": "GO:0006955",
  "gene_symbol": "IGLV2-11",
  "gene": "UniProtKB:P01706",
  "gene_name": "Immunoglobulin lambda variable 2-11"
}